{
  "gene_symbol": "REN",
  "gene": "UniProtKB:P00797",
  "term_id": "GO:0005615",
  "gene_name": "Renin",
  "term_label": "extracellular space"
}